myosin II filament assembly [GO:0031036] (biological process) Definition: The formation of a bipolar filament composed of myosin II molecules. Relationships: is a type of GO:0031034; is a type of myosin II filament organization [GO:0031038] Regulation: regulated by regulation of myosin II filament assembly [GO:0043520]; negatively regulated by negative regulation of myosin II filament assembly [GO:1905510]; positively regulated by positive regulation of myosin II filament assembly [GO:1905511] Also known as: myosin II polymerization Sources: GOC:mah